acinar cell of sebaceous gland differentiation [GO:1903680] (BP) Also known as: sebocyte differentiation Relationships: is_a sebaceous gland cell differentiation [GO:0001949]; is a type of acinar cell differentiation [GO:0090425] References: PMID:17018284, PMID:18334552, PMID:19944183 Sources: GOC:TermGenie, GO_REF:0000086 Definition: The process in which a relatively unspecialized cell acquires the specialized features of an acinar cell of sebaceous gland.